{
  "term_id": "GO:0030018",
  "gene_symbol": "FHL2",
  "gene": "UniProtKB:Q14192",
  "term_label": "Z disc",
  "gene_name": "Four and a half LIM domains protein 2"
}